{
  "term_label": "plasma membrane",
  "gene_symbol": "SLC5A4",
  "gene_name": "Probable glucose sensor protein SLC5A4",
  "gene": "UniProtKB:Q9NY91",
  "term_id": "GO:0005886"
}